{
  "term_label": "plasma membrane",
  "gene_name": "KIR2DL1 protein",
  "gene_symbol": "KIR2DL1",
  "term_id": "GO:0005886",
  "gene": "UniProtKB:A0A5K1VDZ0"
}